{
  "gene_symbol": "CSRNP2",
  "gene": "UniProtKB:Q9H175",
  "gene_name": "Cysteine_serine-rich nuclear protein 2",
  "term_label": "sequence-specific DNA binding",
  "term_id": "GO:0043565"
}